protein-containing complex remodeling [GO:0034367] (biological process) Sources: GOC:BHF, GOC:mah, GOC:mtg_mpo, GOC:rl Definition: The acquisition, loss, or modification of macromolecules within a complex, resulting in the alteration of an existing complex. Relationships: is a type of GO:0043933 Subtypes: protein-DNA-RNA complex remodeling [GO:0001119], protein-DNA complex remodeling [GO:0001120], GO:0034368, protein-RNA complex remodeling [GO:0110136] Also known as: protein-containing complex remodelling, macromolecular complex remodeling, macromolecular complex remodelling